intracellular sodium-activated potassium channel activity [GO:0005228] (MF) References: PMID:12628167 Sources: GOC:mtg_transport Definition: Enables the transmembrane transfer of potassium by a channel that opens in response to stimulus by a sodium ion or ions. Transport by a channel involves facilitated diffusion of a solute (by an energy-independent process) involving passage through a transmembrane aqueous pore or channel, without evidence for a carrier-mediated mechanism. Sodium activated potassium channels have distinctive properties, including a large single channel conductance, subconductance states, and a block of single channel currents at positive potentials, similar to inward rectification. Relationships: is a type of potassium channel activity [GO:0005267]; is a type of monoatomic ion-gated channel activity [GO:0022839]; is a type of ligand-gated monoatomic cation channel activity [GO:0099094] Also known as: intracellular sodium activated potassium channel activity